{
  "gene_symbol": "BRCC3",
  "gene_name": "Lys-63-specific deubiquitinase BRCC36",
  "term_id": "GO:0031593",
  "term_label": "polyubiquitin modification-dependent protein binding",
  "gene": "UniProtKB:P46736"
}